{
  "gene_name": "Uncharacterized protein C12orf71",
  "gene": "UniProtKB:A8MTZ7",
  "term_id": "UNKNOWN:0003",
  "gene_symbol": "C12orf71",
  "term_label": "Unknown cellular component"
}